{
  "gene": "UniProtKB:Q8N3C7",
  "term_id": "GO:0031122",
  "gene_name": "CAP-Gly domain-containing linker protein 4",
  "gene_symbol": "CLIP4",
  "term_label": "cytoplasmic microtubule organization"
}